{
  "term_id": "GO:0012505",
  "term_label": "endomembrane system",
  "gene_name": "Rab-like protein 2A",
  "gene_symbol": "RABL2A",
  "gene": "UniProtKB:Q9UBK7"
}